{
  "gene_symbol": "ID3",
  "gene_name": "DNA-binding protein inhibitor ID-3",
  "term_id": "GO:0030182",
  "term_label": "neuron differentiation",
  "gene": "UniProtKB:Q02535"
}